{
  "gene_symbol": "LYNX1",
  "term_label": "acetylcholine receptor binding",
  "gene_name": "Ly-6_neurotoxin-like protein 1",
  "term_id": "GO:0033130",
  "gene": "UniProtKB:P0DP58"
}